{
  "term_label": "zinc ion transmembrane transport",
  "gene_name": "Probable proton-coupled zinc antiporter SLC30A3",
  "gene": "UniProtKB:Q99726",
  "term_id": "GO:0071577",
  "gene_symbol": "SLC30A3"
}